{
  "term_id": "GO:0003711",
  "gene_name": "Transcription elongation factor A N-terminal and central domain-containing protein 2",
  "term_label": "transcription elongation factor activity",
  "gene_symbol": "TCEANC2",
  "gene": "UniProtKB:Q96MN5"
}